{
  "term_id": "GO:0004984",
  "gene_name": "Olfactory receptor 10G8",
  "gene": "UniProtKB:Q8NGN5",
  "term_label": "olfactory receptor activity",
  "gene_symbol": "OR10G8"
}